{
  "term_id": "UNKNOWN:0001",
  "term_label": "Unknown molecular function",
  "gene_name": "Regulator of G-protein signaling protein-like",
  "gene": "UniProtKB:A5PLK6",
  "gene_symbol": "RGSL1"
}